plastid transcription [GO:0042793] (biological process) Subtypes: GO:0042794 Relationships: is a type of DNA-templated transcription [GO:0006351]; occurs in plastid [GO:0009536] Also known as: transcription from plastid promoter Definition: The synthesis of RNA from a plastid DNA template, usually by a specific plastid RNA polymerase. Sources: GOC:jl, ISBN:0321000382